{
  "term_id": "GO:0003723",
  "gene_symbol": "HNRNPCL2",
  "term_label": "RNA binding",
  "gene_name": "Heterogeneous nuclear ribonucleoprotein C-like 2",
  "gene": "UniProtKB:B2RXH8"
}